neutrophil mediated immunity [GO:0002446] (biological process) Sources: GOC:add, GO_REF:0000022, ISBN:0781735149 Relationships: is a type of myeloid leukocyte mediated immunity [GO:0002444] Definition: Any process involved in the carrying out of an immune response by a neutrophil. Subtypes: neutrophil mediated cytotoxicity [GO:0070942]